regulation of response to alcohol [GO:1901419] (biological process) Subtypes: regulation of response to ethanol [GO:1901416], negative regulation of response to alcohol [GO:1901420], positive regulation of response to alcohol [GO:1901421], GO:1901445, GO:1901448, regulation of cellular response to alcohol [GO:1905957] Relationships: is a type of GO:0048583; regulates response to alcohol [GO:0097305] Sources: GOC:TermGenie, GOC:mengo_curators Definition: Any process that modulates the frequency, rate or extent of response to alcohol.